{
  "gene_name": "Corticotropin-releasing factor receptor 2",
  "gene_symbol": "CRHR2",
  "term_id": "GO:0005886",
  "term_label": "plasma membrane",
  "gene": "UniProtKB:Q13324"
}